{
  "gene": "UniProtKB:P49753",
  "term_label": "Unknown cellular component",
  "gene_symbol": "ACOT2",
  "term_id": "UNKNOWN:0003",
  "gene_name": "Acyl-coenzyme A thioesterase 2, mitochondrial"
}